{
  "term_id": "GO:0048306",
  "gene": "UniProtKB:P29034",
  "gene_name": "Protein S100-A2",
  "gene_symbol": "S100A2",
  "term_label": "calcium-dependent protein binding"
}